{
  "gene_symbol": "GUCY1B2",
  "gene": "UniProtKB:O75343",
  "gene_name": "Guanylate cyclase soluble subunit beta-2",
  "term_label": "guanylate cyclase complex, soluble",
  "term_id": "GO:0008074"
}